{
  "term_id": "GO:1903142",
  "gene": "UniProtKB:P35611",
  "gene_symbol": "ADD1",
  "term_label": "positive regulation of establishment of endothelial barrier",
  "gene_name": "Alpha-adducin"
}